{
  "term_id": "GO:0019899",
  "term_label": "enzyme binding",
  "gene_name": "UDP-glucuronosyltransferase 1A9",
  "gene_symbol": "UGT1A9",
  "gene": "UniProtKB:O60656"
}